{
  "term_id": "GO:0005886",
  "gene_symbol": "OR52A1",
  "gene_name": "Olfactory receptor 52A1",
  "gene": "UniProtKB:Q9UKL2",
  "term_label": "plasma membrane"
}